{
  "term_id": "UNKNOWN:0001",
  "gene_name": "Syntabulin",
  "term_label": "Unknown molecular function",
  "gene_symbol": "SYBU",
  "gene": "UniProtKB:Q9NX95"
}